Golgi cell precursor proliferation [GO:0021926] (biological process) Relationships: is a type of cell proliferation in hindbrain ventricular zone [GO:0021923] References: PMID:15157725 Sources: GOC:cls, GOC:dgh, GOC:dph, GOC:jid, GO_REF:0000021 Definition: The multiplication or reproduction of neuroblasts that will give rise to Golgi cells. A Golgi cell is an inhibitory GABAergic interneuron found in the cerebellar cortex.